{
  "gene_symbol": "CATSPERE",
  "term_id": "GO:0048240",
  "gene": "UniProtKB:Q5SY80",
  "term_label": "sperm capacitation",
  "gene_name": "Cation channel sperm-associated auxiliary subunit epsilon"
}